{
  "term_label": "cell-cell adhesion mediator activity",
  "gene": "UniProtKB:O95484",
  "gene_symbol": "CLDN9",
  "term_id": "GO:0098632",
  "gene_name": "Claudin-9"
}